D-ribulose-phosphate 3-epimerase activity [GO:0004750] (MF) Sources: EC:5.1.3.1, RHEA:13677 Definition: Catalysis of the reaction: D-ribulose 5-phosphate = D-xylulose 5-phosphate. Relationships: is a type of racemase and epimerase activity, acting on carbohydrates and derivatives [GO:0016857] Also known as: D-ribulose 5-phosphate epimerase activity, D-ribulose phosphate-3-epimerase activity, D-ribulose-5-P 3-epimerase activity, D-ribulose-5-phosphate 3-epimerase activity, D-ribulose-5-phosphate epimerase activity, D-xylulose-5-phosphate 3-epimerase activity, erythrose-4-phosphate epimerase activity, erythrose-4-phosphate isomerase activity, pentose phosphate epimerase (PPE), pentose-5-phosphate 3-epimerase activity, phosphoketopentose 3-epimerase activity, phosphoketopentose epimerase activity, phosphoribulose epimerase activity, ribulose 5-phosphate 3-epimerase activity, ribulose-phosphate 3-epimerase activity, xylulose phosphate 3-epimerase activity